cytoskeleton-dependent cytoplasmic transport, nurse cell to oocyte [GO:0019749] (biological process) Definition: The directed movement of substances along cytoskeletal elements, such as microfilaments or microtubules, from a nurse cell to an oocyte. Sources: GOC:ai Relationships: is a type of cytoskeleton-dependent intracellular transport [GO:0030705]